{
  "gene_symbol": "SIM1",
  "term_label": "DNA-binding transcription factor activity, RNA polymerase II-specific",
  "term_id": "GO:0000981",
  "gene_name": "Single-minded homolog 1",
  "gene": "UniProtKB:P81133"
}